isoflavonoid catabolic process [GO:0046288] (biological process) Definition: The chemical reactions and pathways resulting in the breakdown of isoflavonoids, a group of water-soluble phenolic derivatives, isomeric with flavonoids. Sources: GOC:ai Subtypes: isoflavonoid phytoalexin catabolic process [GO:0046290] Relationships: is a type of phenylpropanoid catabolic process [GO:0046271]; is a type of GO:0046287 Also known as: isoflavonoid breakdown, isoflavonoid catabolism, isoflavonoid degradation